APC-IQGAP1-Cdc42 complex [GO:0034744] (cellular component) Note: Note that the gene/protein name 'APC' should not be confused with the abbreviation for 'anaphase promoting complex'. References: PMID:15572129 Definition: A protein complex that contains the tumor suppressor protein adenomatous polyposis coli (APC), the small GTPase Cdc42, and the Rac1 and Cdc42 effector IQGAP1; may play a role in cytoskeleton organization and cell migration. Relationships: is a type of intracellular protein-containing complex [GO:0140535]; is a type of GTPase complex [GO:1905360]; is part of cell leading edge [GO:0031252]